{
  "gene": "UniProtKB:Q14563",
  "term_label": "negative chemotaxis",
  "gene_name": "Semaphorin-3A",
  "term_id": "GO:0050919",
  "gene_symbol": "SEMA3A"
}